{
  "gene_symbol": "SLC3A1",
  "term_id": "GO:0006865",
  "term_label": "amino acid transport",
  "gene_name": "Neutral and basic amino acid transport protein rBAT",
  "gene": "UniProtKB:Q07837"
}